{
  "term_label": "proteasome-mediated ubiquitin-dependent protein catabolic process",
  "gene_symbol": "KLHL20",
  "term_id": "GO:0043161",
  "gene": "UniProtKB:Q9Y2M5",
  "gene_name": "Kelch-like protein 20"
}